{
  "gene_name": "Olfactory receptor 56A4",
  "gene": "UniProtKB:Q8NGH8",
  "term_label": "Unknown biological process",
  "gene_symbol": "OR56A4",
  "term_id": "UNKNOWN:0002"
}